{
  "term_id": "GO:0006357",
  "gene_name": "Zinc finger protein 248",
  "gene_symbol": "ZNF248",
  "term_label": "regulation of transcription by RNA polymerase II",
  "gene": "UniProtKB:Q8NDW4"
}